{
  "term_label": "positive regulation of tumor necrosis factor production",
  "gene_symbol": "FCGR2C",
  "term_id": "GO:0032760",
  "gene_name": "Low affinity immunoglobulin gamma Fc region receptor II-c",
  "gene": "UniProtKB:P31995"
}